{
  "gene": "UniProtKB:O75173",
  "term_id": "GO:0004222",
  "gene_symbol": "ADAMTS4",
  "term_label": "metalloendopeptidase activity",
  "gene_name": "A disintegrin and metalloproteinase with thrombospondin motifs 4"
}